{
  "term_id": "UNKNOWN:0001",
  "gene": "UniProtKB:Q13069",
  "gene_name": "G antigen 5",
  "gene_symbol": "GAGE5",
  "term_label": "Unknown molecular function"
}